{
  "gene_symbol": "MOB3A",
  "gene_name": "MOB kinase activator 3A",
  "gene": "UniProtKB:Q96BX8",
  "term_label": "signal transduction",
  "term_id": "GO:0007165"
}